{
  "term_id": "GO:0016324",
  "gene_name": "V-type proton ATPase subunit B, brain isoform",
  "gene": "UniProtKB:P21281",
  "gene_symbol": "ATP6V1B2",
  "term_label": "apical plasma membrane"
}